{
  "gene": "UniProtKB:O60294",
  "gene_name": "tRNA wybutosine-synthesizing protein 4",
  "term_label": "wybutosine biosynthetic process",
  "gene_symbol": "LCMT2",
  "term_id": "GO:0031591"
}